{
  "term_id": "UNKNOWN:0001",
  "term_label": "Unknown molecular function",
  "gene_symbol": "GATAD1",
  "gene": "UniProtKB:Q8WUU5",
  "gene_name": "GATA zinc finger domain-containing protein 1"
}